GTP diphosphokinase activity [GO:0008728] (molecular function) Sources: EC:2.7.6.5 Relationships: is a type of GO:0016778 Definition: Catalysis of the reaction: ATP + GTP = AMP + guanosine 3'-diphosphate 5'-triphosphate. Also known as: GTP pyrophosphokinase activity, (p)ppGpp synthetase I, (p)ppGpp synthetase II, ATP-GTP 3'-diphosphotransferase activity, ATP:GTP 3'-diphosphotransferase activity, GPSI, GPSII, guanosine 3',5'-polyphosphate synthase activity, guanosine 5',3'-polyphosphate synthetase activity, guanosine pentaphosphate synthetase activity, ppGpp synthetase I activity, stringent factor activity